regulation of lncRNA transcription [GO:0140743] (biological process) References: PMID:33767452, PMID:33913806 Relationships: is a type of regulation of DNA-templated transcription [GO:0006355]; regulates lncRNA transcription [GO:0140742] Definition: Any process that modulates the frequency, rate or extent of the synthesis of a lncRNA. Subtypes: negative regulation of lncRNA transcription [GO:0140744]